chorion development [GO:0060717] (biological process) Relationships: is a type of extraembryonic membrane development [GO:1903867] Definition: The biological process whose specific outcome is the progression of a chorion from an initial condition to its mature state. This process begins with the formation of the structure and ends with the mature structure. The chorion is an extraembryonic membrane. Sources: GOC:dph